{
  "term_label": "Unknown cellular component",
  "gene_symbol": "A0A669KB60",
  "gene": "UniProtKB:A0A669KB60",
  "gene_name": "Uncharacterized protein",
  "term_id": "UNKNOWN:0003"
}